{
  "gene_name": "Phosducin-like protein 3",
  "term_label": "vascular endothelial growth factor receptor 2 binding",
  "gene_symbol": "PDCL3",
  "gene": "UniProtKB:Q9H2J4",
  "term_id": "GO:0043184"
}